 [RO:0002175]